energy homeostasis [GO:0097009] (biological process) Also known as: negative regulation of energy homeostasis, positive regulation of energy homeostasis, regulation of energy homeostasis Relationships: is a type of multicellular organismal-level homeostasis [GO:0048871] Subtypes: GO:0002021 References: PMID:15919751 Sources: GOC:yaf Definition: Any process involved in the balance between food intake (energy input) and energy expenditure.